{
  "term_id": "UNKNOWN:0001",
  "gene": "UniProtKB:Q9BR11",
  "gene_name": "Zinc finger SWIM domain-containing protein 1",
  "term_label": "Unknown molecular function",
  "gene_symbol": "ZSWIM1"
}